{
  "gene": "UniProtKB:Q86WX3",
  "term_label": "Unknown biological process",
  "term_id": "UNKNOWN:0002",
  "gene_name": "Active regulator of SIRT1",
  "gene_symbol": "RPS19BP1"
}